apical junction assembly [GO:0043297] (biological process) Also known as: apical junction complex assembly References: PMID:10854689, PMID:14729475, PMID:15196556 Sources: GOC:go_curators Relationships: is a type of cell-cell junction assembly [GO:0007043] Definition: The formation of an apical junction, a functional unit located near the cell apex at the points of contact between epithelial cells composed of the tight junction, the zonula adherens junction and the desmosomes, by the aggregation, arrangement and bonding together of its constituents.